regulation of B cell differentiation [GO:0045577] (biological process) Subtypes: GO:0001924, regulation of central B cell deletion [GO:0002898], GO:0002914, negative regulation of B cell differentiation [GO:0045578], GO:0045579, regulation of plasma cell differentiation [GO:1900098] Relationships: is a type of regulation of lymphocyte differentiation [GO:0045619]; is a type of regulation of B cell activation [GO:0050864]; regulates GO:0030183 Definition: Any process that modulates the frequency, rate or extent of B cell differentiation. Sources: GOC:go_curators Note: Note that immunologists typically use the word 'development' to refer to cells of B or T cell lineages undergoing the process that GO describes as 'cell differentiation'. Also known as: regulation of B lymphocyte differentiation, regulation of B-cell differentiation, regulation of B-lymphocyte differentiation, regulation of B cell development